histone H3K36me2/H3K36me3 demethylase activity [GO:0140681] (molecular function) Also known as: histone H3K36me2 demethylase activity, histone H3-tri/dimethyl-lysine-36 demethylase activity, histone H3K36me3 demethylase activity Note: Comment: Note that the residue position corresponds to the canonical human H3 histone (UniProtKB:P84243); this residue is conserved across all eukaryotes. Residue 1 is the first residue following removal of the initiating Methionine (Met). Note that each histone is encoded by multiple genes, and sequences may vary across different genes within an organism. References: PMID:21914792 Relationships: is a type of histone H3K36 demethylase activity [GO:0051864] Definition: Catalysis of the removal of a methyl group from a tri- or a dimethyl-lysine residue at position 36 of the histone H3 protein. This is a dioxygenase reaction that is dependent on Fe(II) and 2-oxoglutarate.